{
  "term_label": "Unknown molecular function",
  "gene": "UniProtKB:Q9UMX5",
  "gene_symbol": "NENF",
  "term_id": "UNKNOWN:0001",
  "gene_name": "Neudesin"
}